{
  "gene_name": "HEAT repeat-containing protein 5B",
  "term_id": "GO:0006897",
  "gene_symbol": "HEATR5B",
  "term_label": "endocytosis",
  "gene": "UniProtKB:Q9P2D3"
}